{
  "gene_name": "Large ribosomal subunit protein uL23m",
  "term_id": "GO:0032543",
  "gene_symbol": "MRPL23",
  "gene": "UniProtKB:Q16540",
  "term_label": "mitochondrial translation"
}